{
  "term_label": "regulation of regulatory ncRNA processing",
  "gene_name": "Interferon-inducible double-stranded RNA-dependent protein kinase activator A",
  "gene_symbol": "PRKRA",
  "term_id": "GO:0070920",
  "gene": "UniProtKB:O75569"
}